bacterial-type DNA replication [GO:0044787] (biological process) Definition: The DNA-dependent DNA replication, exemplified by prokaryotes, that occurs as part of the cell cycle. Prokaryotic DNA replication is bi-directional and originates at a single origin of replication on the circular genome. Relationships: is a type of GO:0044786 Sources: GOC:mtg_cell_cycle Also known as: bacterial-type cell cycle DNA replication